{
  "term_id": "GO:0030509",
  "gene_symbol": "BMP10",
  "term_label": "BMP signaling pathway",
  "gene_name": "Bone morphogenetic protein 10",
  "gene": "UniProtKB:O95393"
}